lipid transmembrane transporter activity [GO:0170055] (molecular function) Sources: GOC:curators Relationships: is a type of lipid transporter activity [GO:0005319]; is_a transmembrane transporter activity [GO:0022857] Subtypes: GO:0015125, GO:0015221, fatty acid transmembrane transporter activity [GO:0015245], ATPase-coupled lipid transmembrane transporter activity [GO:0034040], retinol transmembrane transporter activity [GO:0034632], polymyxin transmembrane transporter activity [GO:0042897], GO:0051978, icosanoid transmembrane transporter activity [GO:0071714], abscisic acid transmembrane transporter activity [GO:0090440], isopentenyl pyrophosphate transmembrane transporter activity [GO:0170045], gibberellin transmembrane transporter activity [GO:1905201] Definition: Enables the transfer of a lipid from one side of a membrane to the other.